{
  "gene_symbol": "MAPK11",
  "term_id": "GO:0005634",
  "gene": "UniProtKB:Q15759",
  "gene_name": "Mitogen-activated protein kinase 11",
  "term_label": "nucleus"
}